{
  "gene_symbol": "AIRIM",
  "gene_name": "AFG2-interacting ribosome maturation factor",
  "gene": "UniProtKB:Q9NX04",
  "term_label": "Unknown molecular function",
  "term_id": "UNKNOWN:0001"
}